{
  "term_id": "GO:0007204",
  "term_label": "positive regulation of cytosolic calcium ion concentration",
  "gene_symbol": "ADRA1D",
  "gene_name": "Alpha-1D adrenergic receptor",
  "gene": "UniProtKB:P25100"
}